{
  "term_id": "UNKNOWN:0002",
  "term_label": "Unknown biological process",
  "gene_symbol": "DHX30",
  "gene_name": "ATP-dependent RNA helicase DHX30",
  "gene": "UniProtKB:Q7L2E3"
}